{
  "term_label": "Unknown biological process",
  "gene": "UniProtKB:O95873",
  "gene_symbol": "C6orf47",
  "term_id": "UNKNOWN:0002",
  "gene_name": "Uncharacterized protein C6orf47"
}